{
  "term_id": "GO:0005737",
  "term_label": "cytoplasm",
  "gene": "UniProtKB:Q9NZ72",
  "gene_name": "Stathmin-3",
  "gene_symbol": "STMN3"
}